{
  "gene_name": "Ubiquitin carboxyl-terminal hydrolase 43",
  "gene_symbol": "USP43",
  "gene": "UniProtKB:Q70EL4",
  "term_id": "UNKNOWN:0001",
  "term_label": "Unknown molecular function"
}